photosystem I [GO:0009522] (cellular component) References: PMID:9821949 Sources: GOC:ds, GOC:mah, ISBN:0140514031 Definition: A photosystem that contains an iron-sulfur reaction center associated with accessory pigments and electron carriers. In cyanobacteria and chloroplasts, photosystem I functions as a light-dependent plastocyanin-ferredoxin oxidoreductase, transferring electrons from plastocyanin to ferredoxin; in photosynthetic bacteria that have only a single type I photosystem, such as the green sulfur bacteria, electrons can go either to ferredoxin (Fd) -> NAD+ or to menaquinone (MK) -> Cytb/FeS -> Cytc555 -> photosystem I (cyclic photophosphorylation). Subtypes: chloroplast photosystem I [GO:0030093], plasma membrane-derived photosystem I [GO:0030094] Relationships: is a type of photosystem [GO:0009521]